{
  "gene_name": "Hydroxysteroid dehydrogenase-like protein 2",
  "term_id": "GO:0005739",
  "gene": "UniProtKB:Q6YN16",
  "gene_symbol": "HSDL2",
  "term_label": "mitochondrion"
}